positive regulation of podosome assembly [GO:0071803] (biological process) Definition: Any process that activates or increases the rate or extent of podosome assembly. Sources: GOC:mah, GOC:sl Relationships: is a type of positive regulation of protein-containing complex assembly [GO:0031334]; is a type of regulation of podosome assembly [GO:0071801]; is a type of positive regulation of organelle assembly [GO:1902117]; positively regulates podosome assembly [GO:0071800] Also known as: up regulation of podosome assembly, up-regulation of podosome assembly, upregulation of podosome assembly, activation of podosome assembly, stimulation of podosome assembly